{
  "gene": "UniProtKB:Q9HAS0",
  "gene_symbol": "C17orf75",
  "term_id": "GO:0099041",
  "gene_name": "Protein Njmu-R1",
  "term_label": "vesicle tethering to Golgi"
}